{
  "gene": "UniProtKB:O60870",
  "gene_symbol": "KIN",
  "term_label": "double-stranded DNA binding",
  "gene_name": "DNA_RNA-binding protein KIN17",
  "term_id": "GO:0003690"
}